{
  "gene_name": "Fibroblast growth factor 7",
  "term_id": "GO:0050679",
  "gene_symbol": "FGF7",
  "term_label": "positive regulation of epithelial cell proliferation",
  "gene": "UniProtKB:P21781"
}